neuron development involved in amphid sensory organ development [GO:0003388] (biological process) Definition: The process whose specific outcome is the progression of a neuron over time, that contributes to the development of the amphid sensory organ. Relationships: is a type of neuron development [GO:0048666]; is part of neuron differentiation involved in amphid sensory organ development [GO:0003387] Sources: GOC:ascb_2009, GOC:dph, GOC:tb